{
  "gene_symbol": "ITPR1",
  "term_label": "phosphatidylinositol binding",
  "term_id": "GO:0035091",
  "gene": "UniProtKB:Q14643",
  "gene_name": "Inositol 1,4,5-trisphosphate receptor type 1"
}